negative regulation of protein monoubiquitination [GO:1902526] (biological process) References: PMID:21931591 Sources: GOC:TermGenie Also known as: down regulation of protein monoubiquitination, down regulation of protein monoubiquitinylation, down regulation of protein monoubiquitylation, down-regulation of protein monoubiquitination, down-regulation of protein monoubiquitinylation, down-regulation of protein monoubiquitylation, downregulation of protein monoubiquitination, downregulation of protein monoubiquitinylation, downregulation of protein monoubiquitylation, negative regulation of protein monoubiquitinylation, negative regulation of protein monoubiquitylation, inhibition of protein monoubiquitination, inhibition of protein monoubiquitinylation, inhibition of protein monoubiquitylation Definition: Any process that stops, prevents or reduces the frequency, rate or extent of protein monoubiquitination. Relationships: is a type of negative regulation of protein ubiquitination [GO:0031397]; is a type of GO:1902525; negatively regulates protein monoubiquitination [GO:0006513]